sequence-specific DNA binding [GO:0043565] (molecular function) Definition: Binding to DNA of a specific nucleotide composition, e.g. GC-rich DNA binding, or with a specific sequence motif or type of DNA e.g. promotor binding or rDNA binding. Sources: GOC:jl Also known as: sequence specific DNA binding Relationships: is a type of DNA binding [GO:0003677] Subtypes: methyl-CpG binding [GO:0008327], telomeric DNA binding [GO:0042162], unmethylated CpG binding [GO:0045322], sequence-specific single stranded DNA binding [GO:0098847], DNA loop anchor binding [GO:0141094], sequence-specific double-stranded DNA binding [GO:1990837]